{
  "term_label": "plasma membrane",
  "gene": "UniProtKB:Q8J025",
  "gene_name": "Protein APCDD1",
  "gene_symbol": "APCDD1",
  "term_id": "GO:0005886"
}